L-methionine salvage [GO:0071267] (biological process) Subtypes: GO:0019284, L-methionine salvage from methylthioadenosine [GO:0019509] Relationships: is a type of amino acid salvage [GO:0043102]; is a type of L-methionine biosynthetic process [GO:0071265] Definition: Any process that generates L-methionine from derivatives of it, without de novo synthesis. Sources: GOC:ecd